{
  "gene_symbol": "GNB1",
  "term_label": "signaling receptor complex adaptor activity",
  "gene": "UniProtKB:P62873",
  "term_id": "GO:0030159",
  "gene_name": "Guanine nucleotide-binding protein G(I)_G(S)_G(T) subunit beta-1"
}